{
  "gene_symbol": "ARRDC4",
  "term_label": "ubiquitin-like ligase-substrate adaptor activity",
  "gene_name": "Arrestin domain-containing protein 4",
  "gene": "UniProtKB:Q8NCT1",
  "term_id": "GO:1990756"
}